{
  "gene_name": "Activator of apoptosis harakiri",
  "gene": "UniProtKB:O00198",
  "gene_symbol": "HRK",
  "term_id": "UNKNOWN:0001",
  "term_label": "Unknown molecular function"
}